{
  "gene_symbol": "GRAMD1B",
  "gene_name": "Protein Aster-B",
  "term_label": "cholesterol transfer activity",
  "term_id": "GO:0120020",
  "gene": "UniProtKB:Q3KR37"
}